{
  "term_id": "GO:0003743",
  "gene": "UniProtKB:P46199",
  "gene_name": "Translation initiation factor IF-2, mitochondrial",
  "term_label": "translation initiation factor activity",
  "gene_symbol": "MTIF2"
}